{
  "term_id": "GO:0004984",
  "gene_symbol": "OR1L8",
  "gene": "UniProtKB:Q8NGR8",
  "term_label": "olfactory receptor activity",
  "gene_name": "Olfactory receptor 1L8"
}